{
  "gene_name": "Olfactory receptor 4C13",
  "term_id": "UNKNOWN:0002",
  "gene_symbol": "OR4C13",
  "term_label": "Unknown biological process",
  "gene": "UniProtKB:Q8NGP0"
}